{
  "gene": "UniProtKB:Q6P3W2",
  "term_id": "UNKNOWN:0003",
  "gene_name": "DnaJ homolog subfamily C member 24",
  "term_label": "Unknown cellular component",
  "gene_symbol": "DNAJC24"
}